dextrin transport [GO:0042955] (biological process) Subtypes: GO:0042956 Sources: GOC:jl Definition: The directed movement of dextrin, any one, or the mixture, of the intermediate polysaccharides formed during the hydrolysis of starch, which are dextrorotatory, soluble in water, and precipitable in alcohol, into, out of or within a cell, or between cells, by means of some agent such as a transporter or pore. Relationships: is_a polysaccharide transport [GO:0015774]